{
  "gene_name": "Tudor domain-containing protein 7",
  "gene_symbol": "TDRD7",
  "term_id": "GO:0070306",
  "term_label": "lens fiber cell differentiation",
  "gene": "UniProtKB:Q8NHU6"
}